{
  "term_label": "mitogen-activated protein kinase binding",
  "gene_name": "TNFAIP3-interacting protein 1",
  "term_id": "GO:0051019",
  "gene_symbol": "TNIP1",
  "gene": "UniProtKB:Q15025"
}